{
  "gene_symbol": "CCNT1",
  "gene_name": "Cyclin-T1",
  "term_label": "cyclin/CDK positive transcription elongation factor complex",
  "term_id": "GO:0008024",
  "gene": "UniProtKB:O60563"
}